{
  "gene_symbol": "SLC2A4",
  "gene_name": "Solute carrier family 2, facilitated glucose transporter member 4",
  "term_label": "dehydroascorbic acid transport",
  "term_id": "GO:0070837",
  "gene": "UniProtKB:P14672"
}